sno(s)RNA-containing ribonucleoprotein complex [GO:0005732] (cellular component) Also known as: sRNP, small nucleolar ribonucleoprotein, small nucleolar ribonucleoprotein complex, small ribonucleoprotein, small ribonucleoprotein protein complex, snoRNP Definition: A ribonucleoprotein complex that contains an RNA molecule of the snoRNA family and associated proteins. Many are involved in a step of processing of rRNA molecules: cleavage, 2'-O-methylation, or pseudouridylation, but other RNA types can be targets as well. The majority fall into one of two classes, box C/D type or box H/ACA type, which are conserved across eukaryotes and archaea. Other members include the telomerase RNA and the ribonuclease MRP RNA. References: PMID:17284456 Sources: GOC:krc, GOC:mah, ISBN:0879695897 Relationships: is a type of GO:1990904 Note: Note that 'nucleolar' in the name acronym 'snoRNA' is part of the RNA family designation 'small nucleolar', and does not reflect the location of the complex. Both box C/D type and box H/ACA RNAs are found in Archaea (where they are referred to as sRNAs) as well as in Eukaryota. In eukaryotes, box H/ACA RNAs are found in both nucleolar-localized snoRNP complexes and in Cajal body-localized scaRNP complexes. Subtypes: ribonuclease MRP complex [GO:0000172], box H/ACA RNP complex [GO:0072588], box C/D RNP complex [GO:0170049]